ADP-D-ribose binding [GO:0072570] (molecular function) Relationships: is a type of anion binding [GO:0043168]; is a type of carbohydrate derivative binding [GO:0097367]; is a type of nucleoside phosphate binding [GO:1901265]; is a type of heterocyclic compound binding [GO:1901363] Definition: Binding to ADP-D-ribose, an ADP-aldose having ribose as the aldose fragment. References: PMID:20088964 Sources: GOC:mah, GOC:sart Also known as: ADP-ribose binding Subtypes: mono-ADP-D-ribose binding [GO:0072571]